sperm motility [GO:0097722] (biological process) Sources: GOC:cilia, GOC:krc Definition: Any process involved in the controlled movement of a sperm cell. Subtypes: flagellated sperm motility [GO:0030317], amoeboid sperm motility [GO:0097723] Relationships: is a type of reproductive process [GO:0022414]; is a type of cell motility [GO:0048870] Also known as: sperm movement